{
  "gene_name": "Interferon alpha-4",
  "term_label": "natural killer cell activation involved in immune response",
  "gene_symbol": "IFNA4",
  "gene": "UniProtKB:P05014",
  "term_id": "GO:0002323"
}